{
  "term_label": "brain development",
  "gene_symbol": "GSX1",
  "term_id": "GO:0007420",
  "gene": "UniProtKB:Q9H4S2",
  "gene_name": "GS homeobox 1"
}